{
  "gene": "UniProtKB:Q08722",
  "gene_name": "Leukocyte surface antigen CD47",
  "gene_symbol": "CD47",
  "term_label": "plasma membrane",
  "term_id": "GO:0005886"
}